{
  "gene_name": "Forkhead box protein S1",
  "term_label": "anatomical structure morphogenesis",
  "term_id": "GO:0009653",
  "gene_symbol": "FOXS1",
  "gene": "UniProtKB:O43638"
}